{
  "gene": "UniProtKB:O15020",
  "term_id": "GO:0030864",
  "term_label": "cortical actin cytoskeleton",
  "gene_name": "Spectrin beta chain, non-erythrocytic 2",
  "gene_symbol": "SPTBN2"
}